{
  "term_label": "cytosol",
  "gene_symbol": "PPP4R4",
  "term_id": "GO:0005829",
  "gene": "UniProtKB:Q6NUP7",
  "gene_name": "Serine_threonine-protein phosphatase 4 regulatory subunit 4"
}